{
  "term_label": "DNA-binding transcription factor activity, RNA polymerase II-specific",
  "gene_name": "Zinc finger protein 202",
  "gene": "UniProtKB:O95125",
  "gene_symbol": "ZNF202",
  "term_id": "GO:0000981"
}